{
  "gene": "UniProtKB:P54284",
  "gene_name": "Voltage-dependent L-type calcium channel subunit beta-3",
  "term_label": "calcium ion transport",
  "term_id": "GO:0006816",
  "gene_symbol": "CACNB3"
}